{
  "term_id": "UNKNOWN:0001",
  "gene_symbol": "ATP6V1G3",
  "term_label": "Unknown molecular function",
  "gene_name": "V-type proton ATPase subunit G 3",
  "gene": "UniProtKB:Q96LB4"
}